{
  "term_label": "Unknown cellular component",
  "term_id": "UNKNOWN:0003",
  "gene_name": "Putative TAP2-associated 6.5 kDa polypeptide",
  "gene_symbol": "Q9Y3F1",
  "gene": "UniProtKB:Q9Y3F1"
}